{
  "gene": "UniProtKB:Q9UL18",
  "gene_name": "Protein argonaute-1",
  "term_id": "GO:0003727",
  "term_label": "single-stranded RNA binding",
  "gene_symbol": "AGO1"
}